mitochondrial phosphate ion transmembrane transport [GO:1990547] (BP) References: PMID:9099701 Definition: The process in which a phosphate ion is transported across a mitochondrial membrane, into or out of the mitochondrion. Relationships: is a type of phosphate ion transmembrane transport [GO:0035435]